{
  "term_label": "nucleus",
  "term_id": "GO:0005634",
  "gene_name": "Transcriptional adapter 2-beta",
  "gene_symbol": "TADA2B",
  "gene": "UniProtKB:Q86TJ2"
}